symbiont-containing vacuolar membrane network [GO:0020006] (cellular component) References: PMID:3528173 Sources: GOC:jl Relationships: is a type of cellular anatomical structure [GO:0110165]; BFO_0000050 GO:0020005 Definition: Tubular network of extensions from the symbiont-containing vacuole membrane that protrude into the host cytoplasm. Also known as: parasitophorous vacuolar membrane network, symbiont-containing vacuole membrane network, tubulovesicular network